{
  "term_label": "nucleus",
  "gene": "UniProtKB:Q9Y2G7",
  "gene_name": "Zinc finger protein 30 homolog",
  "gene_symbol": "ZFP30",
  "term_id": "GO:0005634"
}